{
  "term_id": "GO:0003723",
  "gene_name": "Eukaryotic translation initiation factor 4H",
  "gene": "UniProtKB:Q15056",
  "gene_symbol": "EIF4H",
  "term_label": "RNA binding"
}